{
  "term_id": "GO:0004029",
  "gene": "UniProtKB:P51648",
  "term_label": "aldehyde dehydrogenase (NAD+) activity",
  "gene_name": "Aldehyde dehydrogenase family 3 member A2",
  "gene_symbol": "ALDH3A2"
}